{
  "gene": "UniProtKB:P02549",
  "gene_symbol": "SPTA1",
  "gene_name": "Spectrin alpha chain, erythrocytic 1",
  "term_label": "cortical actin cytoskeleton",
  "term_id": "GO:0030864"
}